{
  "gene_name": "Potassium channel subfamily K member 6",
  "term_id": "GO:0071805",
  "gene": "UniProtKB:Q9Y257",
  "term_label": "potassium ion transmembrane transport",
  "gene_symbol": "KCNK6"
}